{
  "gene": "UniProtKB:P22105",
  "gene_name": "Tenascin-X",
  "term_id": "GO:0030155",
  "gene_symbol": "TNXB",
  "term_label": "regulation of cell adhesion"
}